maleylacetoacetate isomerase activity [GO:0016034] (molecular function) Definition: Catalysis of the reaction: 4-maleylacetoacetate = 4-fumarylacetoacetate. Sources: EC:5.2.1.2 Also known as: 4-maleylacetoacetate cis-trans-isomerase activity, maleylacetoacetic isomerase activity, maleylacetone cis-trans-isomerase activity, maleylacetone isomerase activity Relationships: is a type of cis-trans isomerase activity [GO:0016859]